carnitine decarboxylase activity [GO:0047729] (molecular function) Sources: EC:4.1.1.42, RHEA:21576 Relationships: is a type of carboxy-lyase activity [GO:0016831] Definition: Catalysis of the reaction: carnitine + H+ = 2-methylcholine + CO2. Also known as: carnitine carboxy-lyase (2-methylcholine-forming), carnitine carboxy-lyase activity